{
  "gene_symbol": "CCR4",
  "term_id": "GO:0019722",
  "term_label": "calcium-mediated signaling",
  "gene_name": "C-C chemokine receptor type 4",
  "gene": "UniProtKB:P51679"
}